{
  "term_label": "Unknown molecular function",
  "gene_symbol": "Q7L0L9",
  "term_id": "UNKNOWN:0001",
  "gene_name": "Transmembrane protein LOC653160",
  "gene": "UniProtKB:Q7L0L9"
}